{
  "gene_name": "Sarcoplasmic reticulum histidine-rich calcium-binding protein",
  "gene_symbol": "HRC",
  "gene": "UniProtKB:P23327",
  "term_label": "Unknown biological process",
  "term_id": "UNKNOWN:0002"
}